{
  "term_label": "nucleus",
  "gene": "UniProtKB:Q9UN79",
  "gene_symbol": "SOX13",
  "term_id": "GO:0005634",
  "gene_name": "Transcription factor SOX-13"
}